{
  "gene": "UniProtKB:A8MPX8",
  "gene_name": "Protein phosphatase 2C-like domain-containing protein 1",
  "term_id": "GO:0007165",
  "term_label": "signal transduction",
  "gene_symbol": "PP2D1"
}